{
  "gene": "UniProtKB:Q96NI6",
  "term_label": "glutamatergic synapse",
  "gene_name": "Leucine-rich repeat and fibronectin type-III domain-containing protein 5",
  "gene_symbol": "LRFN5",
  "term_id": "GO:0098978"
}